acylglycerol O-acyltransferase activity [GO:0016411] (molecular function) Subtypes: 1-acylglycerol-3-phosphate O-acyltransferase activity [GO:0003841], 2-acylglycerol O-acyltransferase activity [GO:0003846], diacylglycerol O-acyltransferase activity [GO:0004144], mono-olein transacylation activity [GO:0051264], diolein transacylation activity [GO:0051265] Sources: GOC:ai Relationships: is a type of O-acyltransferase activity [GO:0008374] Definition: Catalysis of the transfer of an acyl group to an oxygen atom on the acylglycerol molecule.